{
  "gene_name": "Neuropilin-1",
  "gene_symbol": "NRP1",
  "term_label": "positive regulation of filopodium assembly",
  "term_id": "GO:0051491",
  "gene": "UniProtKB:O14786"
}